histone acetyltransferase activity [GO:0004402] (molecular function) Definition: Catalysis of the reaction: L-lysyl-[histone] + acetyl-CoA = N6-acetyl-L-lysyl-[histone] + CoA + H+. Subtypes: histone H3 acetyltransferase activity [GO:0010484], histone H4 acetyltransferase activity [GO:0010485], histone H2A acetyltransferase activity [GO:0043998], histone H2B acetyltransferase activity [GO:0044013], histone H1 acetyltransferase activity [GO:0160262] Also known as: histone acetylase activity, histone lysine acetyltransferase activity, H2A/H2B histone acetyltransferase activity, H3/H4 histone acetyltransferase activity, H4/H2 histone acetyltransferase activity, H4/H2A acetyltransferase activity, acetyl-CoA:histone acetyltransferase activity, histone acetokinase activity, histone transacetylase activity, nucleosome-histone acetyltransferase activity Regulation: regulated by histone acetyltransferase regulator activity [GO:0035034] References: PMID:19056256 Sources: RHEA:21992 Relationships: is a type of protein-lysine-acetyltransferase activity [GO:0061733]; is a type of histone modifying activity [GO:0140993]